{
  "gene_symbol": "PAK2",
  "gene_name": "Serine_threonine-protein kinase PAK 2",
  "gene": "UniProtKB:Q13177",
  "term_id": "GO:0005737",
  "term_label": "cytoplasm"
}